foot layer [GO:0043670] (cellular component) Also known as: nexine 1 Definition: The inner layer of the ectexine. Relationships: is a type of GO:0110165; is part of ectexine [GO:0043669] References: PMID:28904424